positive regulation of timing of anagen [GO:0051885] (biological process) Sources: GOC:ai, GOC:pr Relationships: is a type of positive regulation of hair follicle maturation [GO:0048818]; is_a regulation of timing of anagen [GO:0051884]; positively regulates anagen [GO:0042640] Definition: Any process that activates or increases the frequency, rate or extent of timing of anagen, the growth phase of the hair cycle. Also known as: activation of anagen, stimulation of anagen, positive regulation of anagen, up regulation of anagen, up-regulation of anagen, upregulation of anagen